methionine metabolic process [GO:0006555] (biological process) Subtypes: methionine biosynthetic process [GO:0009086], L-methionine catabolic process [GO:0009087] Relationships: is a type of GO:0000096; is a type of alpha-amino acid metabolic process [GO:1901605] Definition: The chemical reactions and pathways involving methionine (2-amino-4-(methylthio)butanoic acid), a sulfur-containing, essential amino acid found in peptide linkage in proteins. Also known as: methionine and threonine metabolic process, methionine and threonine metabolism, methionine metabolism Sources: GOC:jl, ISBN:0198506732